autotransporter activity [GO:0015474] (molecular function) Sources: GOC:mtg_transport, ISBN:0815340729, TC:1.B.12.-.- Relationships: is a type of porin activity [GO:0015288] Definition: Transports a passenger protein from the periplasm to the external milieu; the passenger protein and the porin are the N- and C-terminal regions of the same protein, respectively.